{
  "gene_name": "DNA repair protein complementing XP-A cells",
  "gene_symbol": "XPA",
  "gene": "UniProtKB:P23025",
  "term_label": "UV-damage excision repair",
  "term_id": "GO:0070914"
}